{
  "gene_name": "Beta-defensin 128",
  "term_label": "defense response to Gram-negative bacterium",
  "gene_symbol": "DEFB128",
  "gene": "UniProtKB:Q7Z7B8",
  "term_id": "GO:0050829"
}